{
  "term_id": "GO:0004115",
  "gene_name": "cAMP-specific 3',5'-cyclic phosphodiesterase 4C",
  "gene": "UniProtKB:Q08493",
  "term_label": "3',5'-cyclic-AMP phosphodiesterase activity",
  "gene_symbol": "PDE4C"
}